negative regulation of angiotensin-activated signaling pathway [GO:0110062] (biological process) Definition: Any process that stops, prevents, or reduces the frequency, rate or extent of the angiotensin-activated signaling pathway. References: PMID:28784619 Sources: GOC:lf Relationships: is a type of negative regulation of G protein-coupled receptor signaling pathway [GO:0045744]; is a type of GO:0110061; negatively regulates angiotensin-activated signaling pathway [GO:0038166]